{
  "term_label": "steroid dehydrogenase activity",
  "gene": "UniProtKB:P51857",
  "gene_symbol": "AKR1D1",
  "term_id": "GO:0016229",
  "gene_name": "Aldo-keto reductase family 1 member D1"
}